GCH1 complex [GO:0034615] (cellular component) References: PMID:16696853 Definition: A protein complex that possesses GTP cyclohydrolase I activity. In E. coli and human, the complex is a homodecamer, and monomers are catalytically inactive. Also known as: GTP cyclohydrolase I complex Relationships: is a type of intracellular protein-containing complex [GO:0140535]; is_a GO:1902494